sodium ion-transporting V-type ATPase complex [GO:0016474] (cellular component) References: PMID:15802565 Sources: GOC:mah Also known as: sodium-translocating V-type ATPase complex Definition: A sodium ion-transporting two-sector ATPase complex that couples ATP hydrolysis to the transport of sodium ions across a concentration gradient. The complex comprises a membrane sector (V0) that carries out proton transport and a cytoplasmic compartment sector (V1) that catalyzes ATP hydrolysis. Relationships: is a type of sodium ion-transporting two-sector ATPase complex [GO:0016472]